positive regulation of phosphorylation [GO:0042327] (biological process) Definition: Any process that activates or increases the frequency, rate or extent of addition of phosphate groups to a molecule. Relationships: is a type of regulation of phosphorylation [GO:0042325]; is a type of positive regulation of phosphate metabolic process [GO:0045937]; positively regulates GO:0016310 Also known as: up regulation of phosphorylation, up-regulation of phosphorylation, upregulation of phosphorylation, activation of phosphorylation, stimulation of phosphorylation Subtypes: GO:0001934, positive regulation of kinase activity [GO:0033674] Sources: GOC:jl